{
  "gene_name": "Ultra-long-chain fatty acid omega-hydroxylase",
  "gene": "UniProtKB:Q6NT55",
  "gene_symbol": "CYP4F22",
  "term_id": "GO:0005789",
  "term_label": "endoplasmic reticulum membrane"
}